{
  "term_label": "Golgi apparatus",
  "gene": "UniProtKB:Q92673",
  "term_id": "GO:0005794",
  "gene_symbol": "SORL1",
  "gene_name": "Sortilin-related receptor"
}